{
  "gene": "UniProtKB:Q3ZCT1",
  "gene_symbol": "ZNF260",
  "term_label": "nucleus",
  "gene_name": "Zinc finger protein 260",
  "term_id": "GO:0005634"
}